3'-5'-RNA exonuclease activity [GO:0000175] (molecular function) Also known as: 3'-5' exoribonuclease activity, 3'-5'-exoribonuclease activity Subtypes: poly(A)-specific ribonuclease activity [GO:0004535], exoribonuclease II activity [GO:0008859], GO:0044748, GO:1990838 Definition: Catalysis of the sequential cleavage of mononucleotides from a free 3' terminus of an RNA molecule. Relationships: is a type of 3'-5' exonuclease activity [GO:0008408]; is a type of GO:0016896 Sources: GOC:mah, ISBN:0198547684